{
  "gene": "UniProtKB:P83916",
  "gene_name": "Chromobox protein homolog 1",
  "term_id": "GO:0003682",
  "term_label": "chromatin binding",
  "gene_symbol": "CBX1"
}